{
  "gene": "UniProtKB:Q9H4Y5",
  "term_label": "glutathione metabolic process",
  "term_id": "GO:0006749",
  "gene_symbol": "GSTO2",
  "gene_name": "Glutathione S-transferase omega-2"
}